{
  "gene": "UniProtKB:Q8N2R0",
  "term_id": "GO:0048793",
  "gene_name": "Protein odd-skipped-related 2",
  "gene_symbol": "OSR2",
  "term_label": "pronephros development"
}